{
  "gene": "UniProtKB:Q6ZP82",
  "term_id": "GO:0007157",
  "term_label": "heterophilic cell-cell adhesion",
  "gene_name": "Coiled-coil domain-containing protein 141",
  "gene_symbol": "CCDC141"
}